{
  "term_id": "GO:0022841",
  "gene_symbol": "KCNK15",
  "term_label": "potassium ion leak channel activity",
  "gene_name": "Potassium channel subfamily K member 15",
  "gene": "UniProtKB:Q9H427"
}